{
  "term_id": "GO:0003779",
  "term_label": "actin binding",
  "gene_symbol": "CAP1",
  "gene_name": "Adenylyl cyclase-associated protein 1",
  "gene": "UniProtKB:Q01518"
}